{
  "term_label": "protein polyubiquitination",
  "gene_name": "Ubiquitin-conjugating enzyme E2 W",
  "term_id": "GO:0000209",
  "gene": "UniProtKB:Q96B02",
  "gene_symbol": "UBE2W"
}